rough endoplasmic reticulum cisterna [GO:0120083] (cellular component) Definition: A subcompartment of the rough endoplasmic reticulum consisting of lumenal expansion into a flattened, disc-shaped cavity. References: PMID:12112448 Sources: GOC:sl Relationships: is_a cellular anatomical structure [GO:0110165]; is part of rough endoplasmic reticulum [GO:0005791]; is part of endoplasmic reticulum cisternal network [GO:0071781]